{
  "term_label": "Unknown molecular function",
  "gene_name": "Putative uncharacterized protein LOC100129027",
  "gene_symbol": "Q6AWC8",
  "gene": "UniProtKB:Q6AWC8",
  "term_id": "UNKNOWN:0001"
}